regulation of cytotoxic T cell differentiation [GO:0045583] (biological process) Relationships: is a type of regulation of T cell differentiation [GO:0045580]; regulates cytotoxic T cell differentiation [GO:0045065] Subtypes: negative regulation of cytotoxic T cell differentiation [GO:0045584], positive regulation of cytotoxic T cell differentiation [GO:0045585] Also known as: regulation of cytotoxic T lymphocyte differentiation, regulation of cytotoxic T-cell differentiation, regulation of cytotoxic T-lymphocyte differentiation, regulation of cytotoxic T cell development Sources: GOC:go_curators Definition: Any process that modulates the frequency, rate or extent of cytotoxic T cell differentiation. Note: Note that immunologists typically use the word 'development' to refer to cells of B or T cell lineages undergoing the process that GO describes as 'cell differentiation'.